{
  "gene_name": "Mast cell carboxypeptidase A",
  "term_label": "metallocarboxypeptidase activity",
  "term_id": "GO:0004181",
  "gene": "UniProtKB:P15088",
  "gene_symbol": "CPA3"
}